response to mitochondrial depolarisation [GO:0098780] (biological process) Definition: Any process that results in a change in state or activity of a cell (in terms of movement, secretion, enzyme production, gene expression, etc.) in response to the depolarization of one or more mitochondria. Relationships: is a type of cellular response to stress [GO:0033554] Sources: GOC:dos